{
  "gene": "UniProtKB:Q9NYW0",
  "term_label": "Unknown molecular function",
  "gene_symbol": "TAS2R10",
  "term_id": "UNKNOWN:0001",
  "gene_name": "Taste receptor type 2 member 10"
}